polyacyltrehalose biosynthetic process [GO:0097093] (biological process) Also known as: polyacyltrehalose anabolism, polyacyltrehalose biosynthesis, polyacyltrehalose formation, polyacyltrehalose synthesis Relationships: is a type of glycolipid biosynthetic process [GO:0009247] References: PMID:19729090 Sources: GOC:rs Definition: The chemical reactions and pathways resulting in the formation of polyacyltrehalose, a pentaacylated, trehalose-based glycolipid.